{
  "gene": "UniProtKB:P23409",
  "term_id": "GO:0000978",
  "term_label": "RNA polymerase II cis-regulatory region sequence-specific DNA binding",
  "gene_name": "Myogenic factor 6",
  "gene_symbol": "MYF6"
}